{
  "term_label": "protein modification by small protein conjugation",
  "gene": "UniProtKB:Q9H0Y0",
  "gene_name": "Ubiquitin-like-conjugating enzyme ATG10",
  "gene_symbol": "ATG10",
  "term_id": "GO:0032446"
}